{
  "gene_symbol": "NMRK2",
  "term_id": "UNKNOWN:0002",
  "term_label": "Unknown biological process",
  "gene": "UniProtKB:Q9NPI5",
  "gene_name": "Nicotinamide riboside kinase 2"
}